transcription coactivator binding [GO:0001223] (molecular function) Definition: Binding to a transcription coactivator, a protein involved in positive regulation of transcription via protein-protein interactions with transcription factors and other proteins that positively regulate transcription. Transcription coactivators do not bind DNA directly, but rather mediate protein-protein interactions between activating transcription factors and the basal transcription machinery. Also known as: RNA polymerase II transcription coactivator binding Sources: GOC:krc Relationships: is a type of transcription coregulator binding [GO:0001221]